phospholamban complex [GO:1990629] (cellular component) References: PMID:16043693 Sources: GOC:ame Also known as: cardiac phospholamban complex, cardiac PLB complex, cardiac PLN complex Relationships: is a type of membrane protein complex [GO:0098796]; is a type of endoplasmic reticulum protein-containing complex [GO:0140534]; is part of sarcoplasmic reticulum membrane [GO:0033017] Note: An example of this is PLN in human (UniProt symbol P26678) in PMID:16043693 (inferred from direct assay). Definition: A protein complex found as a homopentamer of the phospholamban (PLN) protein in the sarcoplasmic reticulum (SR) membrane of cardiomyocytes. Cardiac PLN is a main determinant of muscle contraction and relaxation, by regulating intracellular calcium levels.